caprolactam catabolic process [GO:0019384] (biological process) Sources: GOC:curators Relationships: is_a GO:0042178; is a type of lactam catabolic process [GO:0072340] Also known as: caprolactam breakdown, caprolactam catabolism, caprolactam degradation Definition: The chemical reactions and pathways resulting in the breakdown of caprolactam, hexahydro-2h-azepin-2-one, a cyclic amide of caproic acid.